{
  "term_label": "homologous chromosome pairing at meiosis",
  "gene_symbol": "RNF212",
  "gene": "UniProtKB:Q495C1",
  "term_id": "GO:0007129",
  "gene_name": "Probable E3 SUMO-protein ligase RNF212"
}